establishment of latency as a circular episome [GO:0075529] (biological process) Definition: A process by which a virus establishes a latent state within its host as an episome, where the viral genome remains silent in the cytoplasm or nucleus as a circular structure. Sources: GOC:jl Also known as: establishment of circular plasmid latency, establishment of latency as a circular plasmid Relationships: is a type of establishment of episomal latency [GO:0075720]